{
  "term_label": "protein-RNA adaptor activity",
  "gene": "UniProtKB:Q14576",
  "term_id": "GO:0140517",
  "gene_symbol": "ELAVL3",
  "gene_name": "ELAV-like protein 3"
}